{
  "gene": "UniProtKB:O60479",
  "term_label": "nucleus",
  "gene_name": "Homeobox protein DLX-3",
  "gene_symbol": "DLX3",
  "term_id": "GO:0005634"
}